{
  "gene": "UniProtKB:Q9NZ81",
  "gene_symbol": "PRR13",
  "term_label": "Unknown biological process",
  "term_id": "UNKNOWN:0002",
  "gene_name": "Proline-rich protein 13"
}